{
  "gene": "UniProtKB:Q969D9",
  "term_id": "GO:0005139",
  "term_label": "interleukin-7 receptor binding",
  "gene_symbol": "TSLP",
  "gene_name": "Thymic stromal lymphopoietin"
}